{
  "term_id": "GO:0005245",
  "gene_name": "Voltage-dependent calcium channel gamma-3 subunit",
  "gene_symbol": "CACNG3",
  "gene": "UniProtKB:O60359",
  "term_label": "voltage-gated calcium channel activity"
}